{
  "term_id": "GO:0005886",
  "gene": "UniProtKB:Q15669",
  "gene_symbol": "RHOH",
  "term_label": "plasma membrane",
  "gene_name": "Rho-related GTP-binding protein RhoH"
}